HLA-E specific inhibitory MHC class Ib receptor activity [GO:0062082] (molecular function) Sources: DOI:10.1002/9780470015902.a0024246 Definition: Combining with a MHC class Ib molecule of the HLA-A subclass to mediate signaling that inhibits activation of a lymphocyte. Relationships: is a type of inhibitory MHC class Ib receptor activity [GO:0062080]